{
  "gene_name": "Single Ig IL-1-related receptor",
  "term_id": "GO:0005886",
  "gene_symbol": "SIGIRR",
  "gene": "UniProtKB:Q6IA17",
  "term_label": "plasma membrane"
}